{
  "gene": "UniProtKB:Q16696",
  "gene_symbol": "CYP2A13",
  "term_label": "oxidoreductase activity, acting on paired donors, with incorporation or reduction of molecular oxygen, reduced flavin or flavoprotein as one donor, and incorporation of one atom of oxygen",
  "gene_name": "Cytochrome P450 2A13",
  "term_id": "GO:0016712"
}